{
  "gene_name": "Glycogen synthase kinase-3 beta",
  "gene_symbol": "GSK3B",
  "term_id": "GO:0010975",
  "term_label": "regulation of neuron projection development",
  "gene": "UniProtKB:P49841"
}